{
  "term_id": "UNKNOWN:0003",
  "gene": "UniProtKB:Q92844",
  "gene_symbol": "TANK",
  "term_label": "Unknown cellular component",
  "gene_name": "TRAF family member-associated NF-kappa-B activator"
}